{
  "term_id": "GO:0005886",
  "gene_symbol": "IRAK1",
  "gene": "UniProtKB:P51617",
  "term_label": "plasma membrane",
  "gene_name": "Interleukin-1 receptor-associated kinase 1"
}